{
  "gene_name": "Polyglutamine-binding protein 1",
  "term_id": "GO:0043021",
  "term_label": "ribonucleoprotein complex binding",
  "gene": "UniProtKB:O60828",
  "gene_symbol": "PQBP1"
}